{
  "gene_name": "von Willebrand factor A domain-containing protein 3A",
  "gene": "UniProtKB:A6NCI4",
  "term_id": "UNKNOWN:0003",
  "term_label": "Unknown cellular component",
  "gene_symbol": "VWA3A"
}